{
  "gene": "UniProtKB:P47813",
  "gene_symbol": "EIF1AX",
  "gene_name": "Eukaryotic translation initiation factor 1A, X-chromosomal",
  "term_id": "GO:0003743",
  "term_label": "translation initiation factor activity"
}